{
  "gene": "UniProtKB:O60384",
  "term_label": "Unknown biological process",
  "term_id": "UNKNOWN:0002",
  "gene_name": "Putative zinc finger protein 861",
  "gene_symbol": "ZNF861P"
}